protein localization involved in auxin polar transport [GO:1901703] (biological process) Definition: Any protein localization that is involved in auxin polar transport. Relationships: is a type of intracellular protein localization [GO:0008104]; is part of auxin polar transport [GO:0009926] Also known as: establishment and maintenance of protein localization involved in auxin polar transport, protein localisation involved in auxin polar transport References: PMID:23163883 Sources: GOC:TermGenie